intracellular accumulation of glycerol [GO:0006973] (biological process) Relationships: is a type of cellular homeostasis [GO:0019725]; BFO_0000050 cellular hyperosmotic response [GO:0071474] References: PMID:11752666 Sources: GOC:jl Definition: The accumulation of glycerol within a cell, for example by increased glycerol biosynthesis combined with decreased permeability of the cell membrane to glycerol, in response to the detection of a hyperosmotic environment.